postsynaptic recycling endosome [GO:0098837] (cellular component) Also known as: postsynaptic endosomal recycling compartment, postsynaptic recycling outpost Relationships: is a type of recycling endosome [GO:0055037]; is a type of GO:0098845 Definition: A recycling endosome of the postsynapse. In postsynaptic terminals with dendritic spines, it is typically located at the base of a dendritic spine. It is involved in recycling of neurotransmitter receptors to the postsynaptic membrane. In some cases at least, this recycling is activated by postsynaptic signaling and so can play a role in long term potentiation. References: PMID:20820847